{
  "term_id": "GO:0006457",
  "gene_name": "Putative protein PTGES3L",
  "gene_symbol": "PTGES3L",
  "term_label": "protein folding",
  "gene": "UniProtKB:E9PB15"
}